{
  "gene_name": "T cell receptor alpha joining 36 (Fragment)",
  "gene": "UniProtKB:A0A087WU04",
  "term_id": "UNKNOWN:0003",
  "gene_symbol": "TRAJ36",
  "term_label": "Unknown cellular component"
}